inhibition of norepinephrine uptake [GO:0051624] (biological process) Definition: Any process that prevents the activation of the directed movement of norepinephrine into a cell. Also known as: inhibition of levarterenol uptake, inhibition of noradrenaline uptake, inhibition of norepinephrine import Relationships: is a type of GO:0051609; is a type of negative regulation of norepinephrine uptake [GO:0051622] Sources: GOC:ai